{
  "term_id": "UNKNOWN:0001",
  "gene": "UniProtKB:Q8NFZ3",
  "term_label": "Unknown molecular function",
  "gene_name": "Neuroligin-4, Y-linked",
  "gene_symbol": "NLGN4Y"
}